{
  "gene_name": "Protein PET100 homolog, mitochondrial",
  "term_label": "unfolded protein binding",
  "gene": "UniProtKB:P0DJ07",
  "term_id": "GO:0051082",
  "gene_symbol": "PET100"
}